{
  "gene": "UniProtKB:P40426",
  "term_id": "GO:0001228",
  "gene_symbol": "PBX3",
  "gene_name": "Pre-B-cell leukemia transcription factor 3",
  "term_label": "DNA-binding transcription activator activity, RNA polymerase II-specific"
}